{
  "gene": "UniProtKB:Q9NY56",
  "gene_name": "Odorant-binding protein 2a",
  "gene_symbol": "OBP2A",
  "term_id": "GO:0005615",
  "term_label": "extracellular space"
}